emodin catabolic process [GO:1900574] (biological process) Definition: The chemical reactions and pathways resulting in the breakdown of emodin. Sources: GOC:TermGenie, GOC:di Also known as: emodin breakdown, emodin catabolism, emodin degradation Relationships: is a type of phenol-containing compound catabolic process [GO:0019336]; is a type of ketone catabolic process [GO:0042182]; is a type of GO:0090487